{
  "term_id": "UNKNOWN:0001",
  "gene_name": "Threonine synthase-like 1",
  "gene_symbol": "THNSL1",
  "term_label": "Unknown molecular function",
  "gene": "UniProtKB:Q8IYQ7"
}